{
  "gene_symbol": "ATP8B2",
  "term_id": "GO:0045332",
  "gene": "UniProtKB:P98198",
  "term_label": "phospholipid translocation",
  "gene_name": "Phospholipid-transporting ATPase ID"
}